{
  "gene": "UniProtKB:P15173",
  "term_id": "GO:0000981",
  "gene_name": "Myogenin",
  "term_label": "DNA-binding transcription factor activity, RNA polymerase II-specific",
  "gene_symbol": "MYOG"
}